guanidinoacetase activity [GO:0047970] (molecular function) Also known as: glycocyaminase activity, guanidinoacetate amidinohydrolase activity Definition: Catalysis of the reaction: guanidinoacetate + H2O = glycine + urea. Relationships: is a type of hydrolase activity, acting on carbon-nitrogen (but not peptide) bonds, in linear amidines [GO:0016813] Sources: EC:3.5.3.2, RHEA:23268